{
  "gene_symbol": "GUCY2D",
  "term_id": "GO:0004383",
  "gene": "UniProtKB:Q02846",
  "term_label": "guanylate cyclase activity",
  "gene_name": "Retinal guanylyl cyclase 1"
}